ionotropic glutamate receptor signaling pathway [GO:0035235] (biological process) Relationships: is a type of glutamate receptor signaling pathway [GO:0007215]; is a type of GO:1990806; has part glutamate-gated receptor activity [GO:0004970] Subtypes: NMDA selective glutamate receptor signaling pathway [GO:0098989], GO:0098990, kainate selective glutamate receptor signaling pathway [GO:0098991] Sources: GOC:signaling, ISBN:0198506732 Definition: The series of molecular signals initiated by glutamate binding to a glutamate receptor on the surface of the target cell, followed by the movement of ions through a channel in the receptor complex, and ending with the regulation of a downstream cellular process, e.g. transcription. Also known as: ionotropic glutamate receptor signalling pathway